{
  "term_id": "GO:0005852",
  "gene_name": "Eukaryotic translation initiation factor 3 subunit C",
  "gene": "UniProtKB:Q99613",
  "gene_symbol": "EIF3C",
  "term_label": "eukaryotic translation initiation factor 3 complex"
}